{
  "gene": "UniProtKB:Q9BVK2",
  "gene_name": "Probable dolichyl pyrophosphate Glc1Man9GlcNAc2 alpha-1,3-glucosyltransferase",
  "gene_symbol": "ALG8",
  "term_id": "GO:0042283",
  "term_label": "dolichyl pyrophosphate Glc1Man9GlcNAc2 alpha-1,3-glucosyltransferase activity"
}